{
  "gene_name": "cAMP-dependent protein kinase type II-alpha regulatory subunit",
  "gene": "UniProtKB:P13861",
  "gene_symbol": "PRKAR2A",
  "term_label": "cAMP-dependent protein kinase inhibitor activity",
  "term_id": "GO:0004862"
}